icosanoid catabolic process [GO:1901523] (biological process) Definition: The chemical reactions and pathways resulting in the breakdown of icosanoid. Sources: GOC:TermGenie, GOC:pr Also known as: icosanoid breakdown, icosanoid catabolism, icosanoid degradation Relationships: is a type of GO:1901569 Subtypes: leukotriene B4 catabolic process [GO:0036101], GO:0062232, F2-isoprostane catabolic process [GO:0062233], leukotriene D4 catabolic process [GO:1901749], leukotriene A4 catabolic process [GO:1901752]